{
  "term_label": "Unknown molecular function",
  "term_id": "UNKNOWN:0001",
  "gene_name": "Sperm protein associated with the nucleus on the X chromosome D",
  "gene_symbol": "SPANXD",
  "gene": "UniProtKB:Q9BXN6"
}